positive regulation of sprouting angiogenesis [GO:1903672] (biological process) Relationships: is a type of positive regulation of angiogenesis [GO:0045766]; is a type of GO:1903670; positively regulates GO:0002040 Definition: Any process that activates or increases the frequency, rate or extent of sprouting angiogenesis. Also known as: up regulation of sprouting angiogenesis, up-regulation of sprouting angiogenesis, upregulation of sprouting angiogenesis, activation of sprouting angiogenesis References: PMID:16756958 Sources: GOC:TermGenie, GO_REF:0000058